4-chlorophenylacetate 3,4-dioxygenase activity [GO:0018622] (molecular function) Sources: EC:1.14.12.9, RHEA:14689 Definition: Catalysis of the reaction: 4-chlorophenylacetate + NADH + O2 = 3,4-dihydroxyphenylacetate + chloride + NAD+. Relationships: is a type of oxidoreductase activity, acting on paired donors, with incorporation or reduction of molecular oxygen, NAD(P)H as one donor, and incorporation of two atoms of oxygen into one donor [GO:0016708] Also known as: 4-chlorophenylacetate,NADH:oxygen oxidoreductase (3,4-hydroxylating, dechlorinating)